{
  "gene_name": "Dynactin subunit 2",
  "gene": "UniProtKB:Q13561",
  "term_label": "Unknown molecular function",
  "gene_symbol": "DCTN2",
  "term_id": "UNKNOWN:0001"
}